phosphatidylinositol-3,5-bisphosphate 3-phosphatase activity [GO:0052629] (MF) Definition: Catalysis of the reaction: 1-phosphatidyl-1D-myo-inositol 3,5-bisphosphate + H2O = 1-phosphatidyl-1D-myo-inositol 5-phosphate + phosphate + 2 H+. References: PMID:19901554 Sources: RHEA:39019 Relationships: is a type of phosphatidylinositol-3,5-bisphosphate phosphatase activity [GO:0106018]